regulation of compound eye photoreceptor development [GO:0045314] (biological process) Also known as: regulation of eye photoreceptor development Sources: GOC:bf Relationships: is a type of regulation of eye photoreceptor cell development [GO:0042478]; is part of regulation of photoreceptor cell differentiation [GO:0046532]; regulates compound eye photoreceptor development [GO:0042051] Subtypes: GO:0045315, negative regulation of compound eye photoreceptor development [GO:0045316] Definition: Any process that modulates the frequency, rate or extent of compound eye photoreceptor development.